{
  "gene_name": "Fructose-bisphosphate aldolase A",
  "term_label": "fructose-bisphosphate aldolase activity",
  "term_id": "GO:0004332",
  "gene_symbol": "ALDOA",
  "gene": "UniProtKB:P04075"
}